sphingolipid floppase activity [GO:0046623] (molecular function) Relationships: is a type of sphingolipid transporter activity [GO:0046624]; is_a floppase activity [GO:0140328]; is part of GO:0099039 Subtypes: ceramide floppase activity [GO:0099038] Also known as: sphingolipid flippase activity, sphingolipid floppase activity (cytosolic to exoplasmic leaflet), sphingolipid-translocating ATPase activity References: PMID:12034738 Sources: GOC:ai Definition: Catalysis of the movement of a sphingolipid from the cytosolic to the exoplasmic leaflet of a membrane, using energy from the hydrolysis of ATP.